interleukin-4-mediated signaling pathway [GO:0035771] (biological process) Also known as: IL-4-mediated signaling pathway, interleukin-4-mediated signalling pathway Relationships: is a type of cytokine-mediated signaling pathway [GO:0019221]; is part of cellular response to interleukin-4 [GO:0071353] Sources: GOC:BHF, GOC:signaling Definition: The series of molecular signals initiated by interleukin-4 binding to its receptor on the surface of a target cell, and ending with the regulation of a downstream cellular process, e.g. transcription. Regulation: regulated by regulation of interleukin-4-mediated signaling pathway [GO:1902214]; negatively regulated by negative regulation of interleukin-4-mediated signaling pathway [GO:1902215]; positively regulated by GO:1902216